{
  "term_label": "cytoplasm",
  "term_id": "GO:0005737",
  "gene_name": "Protein S100-A9",
  "gene": "UniProtKB:P06702",
  "gene_symbol": "S100A9"
}